vacuole-ER tethering [GO:1990854] (biological process) Relationships: is_a GO:0016043; is_a maintenance of ER location [GO:0051685]; is a type of organelle localization by membrane tethering [GO:0140056]; is a type of vacuolar localization [GO:1990849] Also known as: vacuole-ER attachment, vacuole-endoplasmic reticulum attachment, vacuole-endoplasmic reticulum tethering References: PMID:26283797 Definition: The attachment of a lytic vacuole to the endoplasmic reticulum, which may facilitate exchange of metabolites between the organelles.